{
  "gene_symbol": "ADCYAP1R1",
  "gene": "UniProtKB:P41586",
  "term_id": "GO:0017046",
  "term_label": "peptide hormone binding",
  "gene_name": "Pituitary adenylate cyclase-activating polypeptide type I receptor"
}